{
  "term_label": "Unknown cellular component",
  "gene": "UniProtKB:Q86UQ5",
  "term_id": "UNKNOWN:0003",
  "gene_name": "Gilles de la Tourette syndrome chromosomal region candidate gene 1 protein",
  "gene_symbol": "GTSCR1"
}